RNA import into mitochondrion [GO:0035927] (biological process) Definition: The process in which a rRNA, ribosomal ribonucleic acid, is transported from the cytosol into the mitochondrial matrix. References: PMID:20691904 Sources: GOC:ans Also known as: cytoplasmic RNA import into mitochondrion, nuclear-encoded RNA import into mitochondrion Relationships: is a type of RNA transport [GO:0050658]; is a type of GO:0055085 Subtypes: tRNA import into mitochondrion [GO:0016031], rRNA import into mitochondrion [GO:0035928]